{
  "term_label": "nucleus",
  "term_id": "GO:0005634",
  "gene": "UniProtKB:Q00536",
  "gene_name": "Cyclin-dependent kinase 16",
  "gene_symbol": "CDK16"
}